{
  "term_id": "UNKNOWN:0001",
  "term_label": "Unknown molecular function",
  "gene_symbol": "BCAR3",
  "gene": "UniProtKB:O75815",
  "gene_name": "Breast cancer anti-estrogen resistance protein 3"
}